{
  "term_id": "GO:0090307",
  "gene": "UniProtKB:Q7Z460",
  "gene_name": "CLIP-associating protein 1",
  "gene_symbol": "CLASP1",
  "term_label": "mitotic spindle assembly"
}